{
  "term_label": "Unknown cellular component",
  "gene_name": "Ataxin-7-like protein 2",
  "term_id": "UNKNOWN:0003",
  "gene": "UniProtKB:Q5T6C5",
  "gene_symbol": "ATXN7L2"
}